positive regulation of cellular pH reduction [GO:0032849] (biological process) Subtypes: positive regulation of Golgi lumen acidification [GO:1905528] Definition: Any process that activates or increases the frequency, rate, or extent of a process that reduces the internal pH of a cell. Relationships: is a type of GO:0032847; is a type of GO:0048518; is a type of GO:0051452; positively regulates intracellular pH reduction [GO:0051452] Sources: GOC:mah Also known as: positive regulation of cell pH reduction, positive regulation of cellular acidification, positive regulation of intracellular pH reduction, positive regulation of reduction of cellular pH, positive regulation of reduction of pH in cell, up regulation of cellular pH reduction, up-regulation of cellular pH reduction, upregulation of cellular pH reduction, activation of cellular pH reduction, stimulation of cellular pH reduction, positive regulation of intracellular acidification